{
  "gene": "UniProtKB:Q8N9B5",
  "term_label": "nucleus",
  "gene_symbol": "JMY",
  "gene_name": "Junction-mediating and -regulatory protein",
  "term_id": "GO:0005634"
}